{
  "gene_symbol": "DAPK3",
  "term_id": "GO:0043065",
  "gene": "UniProtKB:O43293",
  "term_label": "positive regulation of apoptotic process",
  "gene_name": "Death-associated protein kinase 3"
}